{
  "term_id": "GO:0000447",
  "term_label": "endonucleolytic cleavage in ITS1 to separate SSU-rRNA from 5.8S rRNA and LSU-rRNA from tricistronic rRNA transcript (SSU-rRNA, 5.8S rRNA, LSU-rRNA)",
  "gene_symbol": "ABT1",
  "gene_name": "Activator of basal transcription 1",
  "gene": "UniProtKB:Q9ULW3"
}